{
  "gene_name": "Keratin, type I cytoskeletal 12",
  "term_id": "GO:0005856",
  "gene_symbol": "KRT12",
  "gene": "UniProtKB:Q99456",
  "term_label": "cytoskeleton"
}